{
  "gene_symbol": "ZFPM1",
  "gene_name": "Zinc finger protein ZFPM1",
  "term_id": "GO:0061629",
  "gene": "UniProtKB:Q8IX07",
  "term_label": "RNA polymerase II-specific DNA-binding transcription factor binding"
}